{
  "gene": "UniProtKB:Q92665",
  "gene_name": "Small ribosomal subunit protein mS31",
  "term_label": "Unknown cellular component",
  "gene_symbol": "MRPS31",
  "term_id": "UNKNOWN:0003"
}